{
  "gene_name": "U3 small nucleolar RNA-associated protein 15 homolog",
  "term_label": "nucleolus",
  "gene_symbol": "UTP15",
  "term_id": "GO:0005730",
  "gene": "UniProtKB:Q8TED0"
}